{
  "gene": "UniProtKB:P20337",
  "term_label": "exocytosis",
  "term_id": "GO:0006887",
  "gene_symbol": "RAB3B",
  "gene_name": "Ras-related protein Rab-3B"
}